nucleoside import across plasma membrane [GO:0180015] (biological process) References: PMID:21998139, PMID:30658162 Definition: The directed movement of nucleoside from outside of a cell, across the plasma membrane and into the cytosol. Relationships: is a type of import across plasma membrane [GO:0098739]; is a type of nucleoside transmembrane transport [GO:1901642]